negative cofactor 2 complex [GO:0017054] (cellular component) Definition: A heterodimeric protein complex that can stably associate with TATA-binding protein on promoters, thereby preventing the assembly of transcription factors TFIIA and TFIIB and leading to repression of RNA polymerase II transcription. The two subunits, NC2alpha (Drap1) and NC2beta (Dr1), dimerize through histone fold domains of the H2A/H2B type present in the amino termini. References: PMID:15574413 Relationships: is a type of RNA polymerase II transcription repressor complex [GO:0090571]